{
  "gene_name": "Nucleoredoxin-like protein 1",
  "term_id": "UNKNOWN:0002",
  "gene": "UniProtKB:Q96CM4",
  "term_label": "Unknown biological process",
  "gene_symbol": "NXNL1"
}